pronucleus [GO:0045120] (cellular component) Sources: ISBN:0198506732 Definition: The nucleus of either the ovum or the spermatozoon following fertilization. Thus, in the fertilized ovum, there are two pronuclei, one originating from the ovum, the other from the spermatozoon that brought about fertilization; they approach each other, but do not fuse until just before the first cleavage, when each pronucleus loses its membrane to release its contents. Relationships: is a type of nucleus [GO:0005634] Subtypes: female pronucleus [GO:0001939], male pronucleus [GO:0001940]